response to sucrose [GO:0009744] (biological process) Also known as: response to sucrose stimulus Subtypes: detection of sucrose stimulus [GO:0009731], cellular response to sucrose stimulus [GO:0071329] Definition: Any process that results in a change in state or activity of a cell or an organism (in terms of movement, secretion, enzyme production, gene expression, etc.) as a result of a sucrose stimulus. Relationships: is a type of GO:0034285 Sources: GOC:jl